{
  "term_id": "GO:0030705",
  "gene_symbol": "MYO10",
  "gene": "UniProtKB:Q9HD67",
  "term_label": "cytoskeleton-dependent intracellular transport",
  "gene_name": "Unconventional myosin-X"
}